intracellular pH elevation [GO:0051454] (biological process) Definition: Any process that increases the internal pH of a cell, measured by the concentration of the hydrogen ion. Sources: GOC:ai Subtypes: GO:0035752, phagosome reneutralization [GO:0044655] Also known as: cell pH elevation, cellular alkalinization, elevation of cellular pH, intracellular alkalinization, pH elevation in cell Relationships: is_a regulation of intracellular pH [GO:0051453]